{
  "term_label": "attachment of mitotic spindle microtubules to kinetochore",
  "gene_name": "Chromosome alignment-maintaining phosphoprotein 1",
  "gene": "UniProtKB:Q96JM3",
  "gene_symbol": "CHAMP1",
  "term_id": "GO:0051315"
}